maternal process involved in female pregnancy [GO:0060135] (biological process) Subtypes: maternal placenta development [GO:0001893], mammary gland branching involved in pregnancy [GO:0060745] Sources: GOC:dph Relationships: is a type of multicellular organismal reproductive process [GO:0048609]; is part of female pregnancy [GO:0007565] Definition: A reproductive process occurring in the mother that allows an embryo or fetus to develop within it.